{
  "gene_name": "Dual specificity protein phosphatase 3",
  "gene_symbol": "DUSP3",
  "term_id": "GO:0005737",
  "gene": "UniProtKB:P51452",
  "term_label": "cytoplasm"
}